{
  "term_id": "UNKNOWN:0001",
  "term_label": "Unknown molecular function",
  "gene_symbol": "SSX6P",
  "gene": "UniProtKB:Q7RTT6",
  "gene_name": "Putative protein SSX6"
}